negative regulation of maltopentaose transport [GO:1900316] (biological process) Sources: GOC:TermGenie, GOC:mengo_curators Also known as: down regulation of maltopentaose transport, down-regulation of maltopentaose transport, downregulation of maltopentaose transport, inhibition of maltopentaose transport Relationships: is a type of regulation of maltopentaose transport [GO:1900315]; is a type of GO:1900361; negatively regulates maltopentaose transport [GO:2001101] Definition: Any process that stops, prevents or reduces the frequency, rate or extent of maltopentaose transport.